{
  "gene_name": "Cation-independent mannose-6-phosphate receptor",
  "term_id": "GO:0005770",
  "gene": "UniProtKB:P11717",
  "gene_symbol": "IGF2R",
  "term_label": "late endosome"
}